guanosine phosphorylase activity [GO:0047975] (molecular function) Definition: Catalysis of the reaction: guanosine + phosphate = guanine + D-ribose 1-phosphate. Sources: EC:2.4.2.15 Relationships: is a type of pentosyltransferase activity [GO:0016763] Also known as: guanosine:phosphate D-ribosyltransferase activity, guanosine:phosphate alpha-D-ribosyltransferase activity